{
  "gene_symbol": "MYO1F",
  "gene_name": "Unconventional myosin-If",
  "gene": "UniProtKB:O00160",
  "term_id": "GO:0005737",
  "term_label": "cytoplasm"
}